regulation of B cell chemotaxis [GO:2000537] (biological process) Relationships: is a type of regulation of lymphocyte chemotaxis [GO:1901623]; RO_0002211 B cell chemotaxis [GO:0035754] Sources: GOC:obol Definition: Any process that modulates the frequency, rate or extent of B cell chemotaxis. Subtypes: GO:2000538, negative regulation of B cell chemotaxis [GO:2000550]